{
  "gene_symbol": "TM9SF1",
  "term_label": "Unknown molecular function",
  "gene": "UniProtKB:O15321",
  "term_id": "UNKNOWN:0001",
  "gene_name": "Transmembrane 9 superfamily member 1"
}